histone H2AK15ac reader activity [GO:0140126] (molecular function) Definition: A histone reader that recognizes a histone H2A acetylated at lysine 15. References: PMID:27153538 Note: Note that the residue position corresponds to the canonical human H2A2A histone (UniProtKB:Q6FI13); this residue is conserved across all eukaryotes. Residue 1 is the first residue following removal of the initiating Methionine (Met). Note that each histone is encoded by multiple genes, and sequences may vary across different genes within an organism. Relationships: is a type of histone H2A reader activity [GO:0140054]